AV node cell to bundle of His cell communication by electrical coupling [GO:0086053] (biological process) Also known as: atrioventricular node cell to bundle of His cell communication by electrical coupling Definition: The process that mediates signaling interactions between an AV node cardiomyocyte and a bundle of His cardiac muscle cell by transfer of current between their adjacent cytoplasms via intercellular protein channels. Relationships: is a type of cell communication by electrical coupling involved in cardiac conduction [GO:0086064]; is a type of AV node cell to bundle of His cell communication [GO:0086067] Sources: GOC:BHF, GOC:dph, GOC:mtg_cardiac_conduct_nov11